{
  "term_label": "Unknown cellular component",
  "gene": "UniProtKB:Q8WXH4",
  "gene_name": "Ankyrin repeat and SOCS box protein 11",
  "gene_symbol": "ASB11",
  "term_id": "UNKNOWN:0003"
}